{
  "gene_symbol": "CNTN5",
  "gene": "UniProtKB:O94779",
  "gene_name": "Contactin-5",
  "term_id": "GO:0007411",
  "term_label": "axon guidance"
}